{
  "term_label": "negative regulation of T cell activation",
  "gene_name": "Dual specificity protein phosphatase 3",
  "term_id": "GO:0050868",
  "gene": "UniProtKB:P51452",
  "gene_symbol": "DUSP3"
}